{
  "gene_symbol": "RPS18",
  "term_id": "UNKNOWN:0002",
  "term_label": "Unknown biological process",
  "gene_name": "Small ribosomal subunit protein uS13",
  "gene": "UniProtKB:P62269"
}